{
  "term_label": "Unknown molecular function",
  "term_id": "UNKNOWN:0001",
  "gene_symbol": "PYROXD2",
  "gene": "UniProtKB:Q8N2H3",
  "gene_name": "Pyridine nucleotide-disulfide oxidoreductase domain-containing protein 2"
}